club cell differentiation [GO:0060486] (biological process) Also known as: Clara cell differentiation References: PMID:28144783 Sources: GOC:dph, GOC:mtg_lung Relationships: is a type of GO:0060487 Definition: The process in which a relatively unspecialized cell acquires specialized features of a club cell. A club cell is an unciliated epithelial cell found in the respiratory and terminal bronchioles.